{
  "gene_symbol": "EME1",
  "gene": "UniProtKB:Q96AY2",
  "term_id": "GO:0031573",
  "gene_name": "Crossover junction endonuclease EME1",
  "term_label": "mitotic intra-S DNA damage checkpoint signaling"
}